{
  "term_id": "UNKNOWN:0001",
  "term_label": "Unknown molecular function",
  "gene_name": "Tetraspanin-9",
  "gene": "UniProtKB:O75954",
  "gene_symbol": "TSPAN9"
}